{
  "gene": "UniProtKB:Q19T08",
  "term_id": "GO:2000353",
  "gene_symbol": "ECSCR",
  "term_label": "positive regulation of endothelial cell apoptotic process",
  "gene_name": "Endothelial cell-specific chemotaxis regulator"
}